{
  "gene": "UniProtKB:Q96NA8",
  "gene_name": "t-SNARE domain-containing protein 1",
  "term_label": "vesicle fusion",
  "gene_symbol": "TSNARE1",
  "term_id": "GO:0006906"
}